{
  "term_id": "GO:0015671",
  "gene": "UniProtKB:P02100",
  "gene_symbol": "HBE1",
  "term_label": "oxygen transport",
  "gene_name": "Hemoglobin subunit epsilon"
}